spinal cord commissural neuron specification [GO:0021518] (biological process) Relationships: is a type of neuron fate specification [GO:0048665]; is part of commissural neuron differentiation in spinal cord [GO:0021528] Definition: The process in which a cell becomes capable of differentiating autonomously into a commissural neuron in an environment that is neutral with respect to the developmental pathway. Sources: GOC:cls, GOC:dgh, GOC:dph, GOC:jid, GO_REF:0000021